{
  "gene": "UniProtKB:Q969Q4",
  "term_label": "GTP binding",
  "term_id": "GO:0005525",
  "gene_name": "ADP-ribosylation factor-like protein 11",
  "gene_symbol": "ARL11"
}